{
  "gene_name": "Flotillin-1",
  "gene": "UniProtKB:O75955",
  "gene_symbol": "FLOT1",
  "term_id": "GO:0002020",
  "term_label": "protease binding"
}